serotonin-gated monoatomic cation channel activity [GO:0022850] (molecular function) Also known as: serotonin-gated cation-selective channel activity, serotonin-activated cation-selective channel activity, serotonin-gated monoatomic cation-selective channel activity, 5-hydroxytryptamine-gated receptor-channel, serotonin-gated cation channel activity References: PMID:12867984 Sources: GOC:mtg_transport Note: Note that this term represents an activity and not a gene product. Consider also annotating to the molecular function term 'G protein-coupled serotonin receptor activity ; GO:0004993'. Definition: Enables the transmembrane transfer of a cation by a channel that opens when serotonin has been bound by the channel complex or one of its constituent parts. Relationships: is a type of GO:0022824; is a type of GO:0099094; is a type of serotonin receptor activity [GO:0099589]; is part of GO:0007210